{
  "term_id": "GO:0048471",
  "gene_name": "Heat shock protein HSP 90-alpha",
  "term_label": "perinuclear region of cytoplasm",
  "gene": "UniProtKB:P07900",
  "gene_symbol": "HSP90AA1"
}